striatal medium spiny neuron differentiation [GO:0021773] (biological process) Definition: The process in which a relatively unspecialized cell acquires specialized features of a medium spiny neuron residing in the striatum. Relationships: is a type of forebrain neuron differentiation [GO:0021879]; is a type of GABAergic neuron differentiation [GO:0097154]; is part of striatum development [GO:0021756] Also known as: medium-sized spiny neuron differentiation, striatal MSN differentiation Sources: GOC:cls, GOC:dgh, GOC:dph, GOC:jid, GO_REF:0000021